{
  "term_label": "Unknown biological process",
  "gene_symbol": "IL25",
  "gene": "UniProtKB:Q9H293",
  "term_id": "UNKNOWN:0002",
  "gene_name": "Interleukin-25"
}